{
  "term_id": "GO:0007268",
  "gene": "UniProtKB:Q15700",
  "gene_symbol": "DLG2",
  "term_label": "chemical synaptic transmission",
  "gene_name": "Disks large homolog 2"
}